epistomal sclerite morphogenesis [GO:0048719] (biological process) Sources: GOC:rc Definition: The process in which the anatomical structures of the epistomal sclerite are generated and organized. Relationships: is a type of post-embryonic animal morphogenesis [GO:0009886]; is part of GO:0007453; is part of epistomal sclerite development [GO:0048724]